{
  "term_label": "ATPase-coupled monoatomic cation transmembrane transporter activity",
  "gene_name": "Polyamine-transporting ATPase 13A3",
  "term_id": "GO:0019829",
  "gene": "UniProtKB:Q9H7F0",
  "gene_symbol": "ATP13A3"
}